{
  "gene_name": "Beta-defensin 103",
  "gene": "UniProtKB:P81534",
  "term_label": "defense response to bacterium",
  "gene_symbol": "DEFB103B",
  "term_id": "GO:0042742"
}